{
  "gene": "UniProtKB:Q9Y3L5",
  "term_id": "GO:0005886",
  "gene_name": "Ras-related protein Rap-2c",
  "term_label": "plasma membrane",
  "gene_symbol": "RAP2C"
}